NAD+-protein-cysteine ADP-ribosyltransferase activity [GO:0140803] (molecular function) Definition: Catalysis of the reaction: L-cysteinyl-[protein] + NAD+ = H+ + nicotinamide + S-(ADP-D-ribosyl)-L-cysteinyl-[protein]. References: PMID:25043379 Sources: RHEA:56612 Relationships: is a type of NAD+-protein mono-ADP-ribosyltransferase activity [GO:1990404]